{
  "gene_symbol": "DCAF15",
  "term_id": "GO:0080008",
  "gene_name": "DDB1- and CUL4-associated factor 15",
  "gene": "UniProtKB:Q66K64",
  "term_label": "Cul4-RING E3 ubiquitin ligase complex"
}